{
  "term_label": "nucleus",
  "gene_name": "Dual specificity protein phosphatase 4",
  "gene": "UniProtKB:Q13115",
  "term_id": "GO:0005634",
  "gene_symbol": "DUSP4"
}